{
  "gene": "UniProtKB:P00748",
  "gene_symbol": "F12",
  "gene_name": "Coagulation factor XII",
  "term_label": "serine-type endopeptidase activity",
  "term_id": "GO:0004252"
}